histone H3 demethylase activity [GO:0141052] (molecular function) Relationships: is a type of histone demethylase activity [GO:0032452] References: PMID:17947579 Subtypes: histone H3K4 demethylase activity [GO:0032453], histone H3K9 demethylase activity [GO:0032454], histone H3R2 demethylase activity [GO:0033746], histone H3K36 demethylase activity [GO:0051864], GO:0071558, histone H3K56me2/H3K56me3 demethylase activity [GO:0140760] Definition: Catalysis of the removal of a methyl group from a modified lysine residue of the histone H3 protein. This is a dioxygenase reaction that is dependent on Fe(II) and 2-oxoglutarate.